{
  "term_label": "nucleus",
  "gene_name": "Annexin A6",
  "gene": "UniProtKB:P08133",
  "term_id": "GO:0005634",
  "gene_symbol": "ANXA6"
}